protease inhibitor complex [GO:0097179] (cellular component) Subtypes: serine protease inhibitor complex [GO:0097180] Also known as: peptidase inhibitor complex References: PMID:6323392 Sources: GOC:ans Definition: A heterodimeric protein complex that contains a protease inhibitor and a protease; formation of the complex inhibits protease activity. Relationships: is a type of peptidase inhibitor complex [GO:1904090]